{
  "gene_name": "Zinc finger protein 57 homolog",
  "term_id": "GO:0000981",
  "gene": "UniProtKB:Q9NU63",
  "term_label": "DNA-binding transcription factor activity, RNA polymerase II-specific",
  "gene_symbol": "ZFP57"
}